{
  "gene_name": "Diacylglycerol kinase beta",
  "gene_symbol": "DGKB",
  "gene": "UniProtKB:Q9Y6T7",
  "term_label": "intracellular signal transduction",
  "term_id": "GO:0035556"
}